hyphopodium formation [GO:0075187] (biological process) Definition: The process in which a specialized structure, consisted of stalked, thick-walled, lobed cells of vegetative epiphytic hyphae, is formed, to attach and penetrate the host surface. The host is defined as the larger of the organisms involved in a symbiotic interaction. Relationships: is a type of formation of infection structure [GO:0075015] Also known as: hyphopodium formation on or near host Sources: GOC:pamgo_curators Regulation: regulated by regulation of hyphopodium formation [GO:0075188]; positively regulated by positive regulation of hyphopodium formation [GO:0075189]; RO_0002212 by GO:0075190